{
  "term_label": "Unknown molecular function",
  "gene_name": "MOB-like protein phocein",
  "gene": "UniProtKB:Q9Y3A3",
  "term_id": "UNKNOWN:0001",
  "gene_symbol": "MOB4"
}